intermediate filament [GO:0005882] (cellular component) Subtypes: lamin filament [GO:0005638], neurofilament [GO:0005883], keratin filament [GO:0045095], type III intermediate filament [GO:0045098], glial filament [GO:0097426] References: PMID:17493611, PMID:17551517, PMID:7979242 Sources: ISBN:0198506732 Also known as: intermediate filament associated protein, type I intermediate filament associated protein, type II intermediate filament associated protein Definition: A cytoskeletal structure that forms a distinct elongated structure, characteristically 10 nm in diameter, that occurs in the cytoplasm of eukaryotic cells. Intermediate filaments form a fibrous system, composed of chemically heterogeneous subunits and involved in mechanically integrating the various components of the cytoplasmic space. Intermediate filaments may be divided into five chemically distinct classes: Type I, acidic keratins; Type II, basic keratins; Type III, including desmin, vimentin and others; Type IV, neurofilaments and related filaments; and Type V, lamins. Relationships: is a type of GO:0099513; is part of intermediate filament cytoskeleton [GO:0045111]